{
  "term_id": "GO:0006357",
  "gene_name": "Zinc finger protein 471",
  "gene": "UniProtKB:Q9BX82",
  "term_label": "regulation of transcription by RNA polymerase II",
  "gene_symbol": "ZNF471"
}